{
  "gene": "UniProtKB:Q8NCU8",
  "gene_symbol": "MTLN",
  "gene_name": "Mitoregulin",
  "term_id": "GO:0051284",
  "term_label": "positive regulation of sequestering of calcium ion"
}